regulation of starch utilization system complex assembly [GO:1900512] (biological process) Definition: Any process that modulates the frequency, rate or extent of starch utilization system complex assembly. Also known as: regulation of SUS complex assembly, regulation of assembly of starch utilization system complex Sources: GOC:TermGenie, GOC:mengo_curators Subtypes: negative regulation of starch utilization system complex assembly [GO:1900513], positive regulation of starch utilization system complex assembly [GO:1900514] Relationships: is a type of regulation of protein-containing complex assembly [GO:0043254]; regulates starch utilization system complex assembly [GO:0044574]